{
  "gene_name": "Histone H2A",
  "term_label": "nucleosome",
  "gene": "UniProtKB:A0A8Q3WKH5",
  "gene_symbol": "H2AL1Q",
  "term_id": "GO:0000786"
}